{
  "term_id": "UNKNOWN:0001",
  "gene": "UniProtKB:Q9P0M4",
  "gene_symbol": "IL17C",
  "gene_name": "Interleukin-17C",
  "term_label": "Unknown molecular function"
}